glutamatergic synapse [GO:0098978] (cellular component) Sources: GOC:dos Subtypes: asymmetric, glutamatergic, excitatory synapse [GO:0098985] Relationships: is a type of synapse [GO:0045202] Definition: A synapse that uses glutamate as a neurotransmitter.